{
  "term_label": "Unknown molecular function",
  "gene_symbol": "SMIM24",
  "gene_name": "Small integral membrane protein 24",
  "gene": "UniProtKB:O75264",
  "term_id": "UNKNOWN:0001"
}